{
  "term_id": "GO:0004438",
  "term_label": "phosphatidylinositol-3-phosphate phosphatase activity",
  "gene_symbol": "MTMR6",
  "gene_name": "Myotubularin-related protein 6",
  "gene": "UniProtKB:Q9Y217"
}